rough endoplasmic reticulum [GO:0005791] (cellular component) Definition: The rough (or granular) endoplasmic reticulum (ER) has ribosomes adhering to the outer surface; the ribosomes are the site of translation of the mRNA for those proteins which are either to be retained within the cisternae (ER-resident proteins), the proteins of the lysosomes, or the proteins destined for export from the cell. Glycoproteins undergo their initial glycosylation within the cisternae. Sources: ISBN:0198506732 Also known as: RER, rough ER Relationships: is a type of endoplasmic reticulum [GO:0005783]